{
  "gene_symbol": "KCNS1",
  "term_id": "GO:0001508",
  "gene_name": "Potassium voltage-gated channel subfamily S member 1",
  "gene": "UniProtKB:Q96KK3",
  "term_label": "action potential"
}